heparan-alpha-glucosaminide N-acetyltransferase activity [GO:0015019] (MF) Definition: Catalysis of the reaction: alpha-D-glucosaminyl-[heparan sulfate](n) + acetyl-CoA = N-acetyl-alpha-D-glucosaminyl-[heparan sulfate](n) + CoA + H+. Sources: RHEA:15125 Relationships: is a type of N-acetyltransferase activity [GO:0008080] Also known as: acetyl-CoA:alpha-glucosaminide N-acetyltransferase activity, acetyl-CoA:heparan-alpha-D-glucosaminide N-acetyltransferase activity, heparin-alpha-glucosaminide N-acetyltransferase activity